{
  "gene_symbol": "FOSL1",
  "term_id": "GO:0006357",
  "term_label": "regulation of transcription by RNA polymerase II",
  "gene_name": "Fos-related antigen 1",
  "gene": "UniProtKB:P15407"
}